IgD immunoglobulin complex, GPI-anchored [GO:0071741] (cellular component) Also known as: GPI-anchored IgD Definition: A protein complex composed of two identical immunoglobulin heavy chains of the IgD isotype and two identical immunoglobulin light chains, held together by disulfide bonds, and bound via a GPI-anchor to the plasma membrane of B cells. References: PMID:11282392 Sources: GOC:add, ISBN:0781765196 Note: Note that an IgD immunoglobulin complex has the function of antigen binding if a suitable antigen is available. Relationships: is a type of IgD immunoglobulin complex [GO:0071738]